{
  "gene_name": "Zinc finger protein 562",
  "term_label": "RNA polymerase II cis-regulatory region sequence-specific DNA binding",
  "gene_symbol": "ZNF562",
  "term_id": "GO:0000978",
  "gene": "UniProtKB:Q6V9R5"
}